{
  "gene_symbol": "RPS15",
  "term_id": "GO:0022627",
  "term_label": "cytosolic small ribosomal subunit",
  "gene_name": "Small ribosomal subunit protein uS19",
  "gene": "UniProtKB:P62841"
}